amyloplast organization [GO:0009660] (biological process) Sources: GOC:jid Relationships: is a type of plastid organization [GO:0009657] Also known as: amyloplast organisation, amyloplast organization and biogenesis Definition: A process that is carried out at the cellular level which results in the assembly, arrangement of constituent parts, or disassembly of an amyloplast. An amyloplast is a plastid whose main function is to synthesize and store starch.